{
  "gene_symbol": "PRO3102",
  "term_label": "Unknown cellular component",
  "term_id": "UNKNOWN:0003",
  "gene": "UniProtKB:Q9H379",
  "gene_name": "Putative uncharacterized protein PRO3102"
}